{
  "gene_name": "Splicing regulator ARVCF",
  "gene_symbol": "ARVCF",
  "gene": "UniProtKB:O00192",
  "term_label": "adherens junction",
  "term_id": "GO:0005912"
}